{
  "gene_symbol": "RPAIN",
  "gene": "UniProtKB:Q86UA6",
  "term_label": "Unknown molecular function",
  "term_id": "UNKNOWN:0001",
  "gene_name": "RPA-interacting protein"
}